{
  "gene_symbol": "MGAT2",
  "gene": "UniProtKB:Q10469",
  "term_label": "alpha-1,6-mannosylglycoprotein 2-beta-N-acetylglucosaminyltransferase activity",
  "term_id": "GO:0008455",
  "gene_name": "Alpha-1,6-mannosyl-glycoprotein 2-beta-N-acetylglucosaminyltransferase"
}